formation of growth cone in injured axon [GO:0048689] (biological process) Relationships: is a type of sprouting of injured axon [GO:0048682] Sources: GOC:dgh, GOC:dph, GOC:jid, GOC:lm Regulation: regulated by regulation of formation of growth cone in injured axon [GO:1905942]; negatively regulated by GO:1905943; positively regulated by GO:1905944 Definition: The formation of a growth cone in an injured axon.